{
  "term_label": "positive regulation of protein targeting to mitochondrion",
  "term_id": "GO:1903955",
  "gene": "UniProtKB:Q9P0U1",
  "gene_symbol": "TOMM7",
  "gene_name": "Mitochondrial import receptor subunit TOM7 homolog"
}